{
  "term_id": "GO:0005789",
  "term_label": "endoplasmic reticulum membrane",
  "gene_symbol": "GDPD1",
  "gene_name": "Lysophospholipase D GDPD1",
  "gene": "UniProtKB:Q8N9F7"
}